adenylate cyclase-modulating G protein-coupled receptor signaling pathway [GO:0007188] (biological process) Sources: GOC:mah, GOC:signaling, ISBN:0815316194 Subtypes: GO:0007189, adenylate cyclase-inhibiting G protein-coupled receptor signaling pathway [GO:0007193] Also known as: G protein signaling, coupled to cAMP nucleotide second messenger, G protein signaling, coupled to cyclic AMP nucleotide second messenger, G protein signalling, coupled to cAMP nucleotide second messenger, G protein signalling, coupled to cyclic AMP nucleotide second messenger, G-protein signaling, coupled to cAMP nucleotide second messenger, G-protein signaling, coupled to cyclic AMP nucleotide second messenger, G-protein signalling, coupled to cAMP nucleotide second messenger, G-protein signalling, coupled to cyclic AMP nucleotide second messenger, GPCR signaling pathway via cAMP second messenger, GPCR signaling pathway via modulation of adenylate cyclase activity, adenylate cyclase-modulating GPCR signaling pathway Definition: A G protein-coupled receptor signaling pathway in which the signal is transmitted via the activation or inhibition of adenylyl cyclase activity and a subsequent change in the intracellular concentration of cyclic AMP (cAMP). Relationships: is a type of G protein-coupled receptor signaling pathway [GO:0007186]; has part GO:0004016 Note: This term is intended to cover steps in a GPCR signaling pathway both upstream and downstream of adenylate-cyclase activity. For steps upstream of adenylate cyclase activity, consider instead annotating to 'regulation of adenylate cyclase activity involved in G protein-coupled receptor signaling pathway ; GO:0010578.